{
  "gene": "UniProtKB:P61764",
  "gene_name": "Syntaxin-binding protein 1",
  "term_id": "GO:0006904",
  "term_label": "vesicle docking involved in exocytosis",
  "gene_symbol": "STXBP1"
}